{
  "gene": "UniProtKB:Q8TCS8",
  "gene_symbol": "PNPT1",
  "term_id": "GO:0004654",
  "term_label": "polyribonucleotide nucleotidyltransferase activity",
  "gene_name": "Polyribonucleotide nucleotidyltransferase 1, mitochondrial"
}